{
  "gene": "UniProtKB:Q9UJA3",
  "term_label": "single-stranded DNA helicase activity",
  "term_id": "GO:0017116",
  "gene_symbol": "MCM8",
  "gene_name": "DNA helicase MCM8"
}